{
  "gene": "UniProtKB:Q99457",
  "gene_name": "Nucleosome assembly protein 1-like 3",
  "term_id": "GO:0000785",
  "term_label": "chromatin",
  "gene_symbol": "NAP1L3"
}